fusion of viral membrane with host outer nuclear membrane [GO:0039700] (biological process) Definition: Fusion of a viral primary envelope with the host outer nuclear membrane during nuclear egress. The transitory primary envelope is acquired by the virus as it buds at the inner nuclear membrane and gains access to the perinuclear space. This membrane is lost by fusing with the host outer nuclear membrane during nuclear exit. References: PMID:23057731 Sources: UniProtKB-KW:KW-1181 Also known as: fusion of viral membrane with host outer nuclear membrane involved in nuclear egress, viral primary envelope fusion with host outer nuclear membrane Relationships: is a type of GO:0016032; is part of exit of virus from host cell nucleus by nuclear egress [GO:0046802]